vitamin-K-epoxide reductase (warfarin-insensitive) activity [GO:0047058] (molecular function) Definition: Catalysis of the reaction: 3-hydroxy-2-methyl-3-phytyl-2,3-dihydronaphthoquinone + oxidized dithiothreitol + H2O = 2,3-epoxy-2,3-dihydro-2-methyl-3-phytyl-1,4-naphthoquinone + 1,4-dithiothreitol. Relationships: is a type of oxidoreductase activity, acting on CH or CH2 groups, disulfide as acceptor [GO:0016728] Also known as: vitamin K 2,3-epoxide reductase activity Sources: RHEA:21560